{
  "term_label": "regulation of gene expression",
  "gene": "UniProtKB:Q495X7",
  "gene_symbol": "TRIM60",
  "term_id": "GO:0010468",
  "gene_name": "Tripartite motif-containing protein 60"
}